{
  "term_label": "DNA 5-methylcytosine dioxygenase activity",
  "gene_name": "Methylcytosine dioxygenase TET2",
  "gene": "UniProtKB:Q6N021",
  "gene_symbol": "TET2",
  "term_id": "GO:0070579"
}